Spemann organizer formation at the embryonic shield [GO:0060063] (biological process) Relationships: is a type of Spemann organizer formation [GO:0060061] Note: Occurs in Teleost fish. Also known as: Spemann's organizer formation at the embryonic shield, Spemann-Mangold organizer formation at the embryonic shield Definition: Formation of the specialized region of the embryonic shield of the embryo that acts as the main signaling center establishing the teleost body plan. References: PMID:9442883 Sources: GOC:dph